{
  "gene_name": "Ran guanine nucleotide release factor",
  "gene": "UniProtKB:Q9HD47",
  "term_id": "GO:0005634",
  "gene_symbol": "RANGRF",
  "term_label": "nucleus"
}